{
  "gene": "UniProtKB:Q9Y289",
  "gene_symbol": "SLC5A6",
  "term_label": "sodium-dependent multivitamin transmembrane transporter activity",
  "gene_name": "Sodium-dependent multivitamin transporter",
  "term_id": "GO:0008523"
}